choline biosynthetic process [GO:0042425] (biological process) Subtypes: choline biosynthetic process via CDP-choline [GO:0033323], choline biosynthetic process via N-monomethylethanolamine [GO:0033324], choline biosynthetic process via phosphoryl-ethanolamine [GO:0033325] Relationships: is a type of GO:0019695; is a type of biogenic amine biosynthetic process [GO:0042401] Sources: GOC:jl, ISBN:0192801023 Also known as: choline anabolism, choline biosynthesis, choline formation, choline synthesis Definition: The chemical reactions and pathways resulting in the formation of choline (2-hydroxyethyltrimethylammonium), an amino alcohol that occurs widely in living organisms as a constituent of certain types of phospholipids and in the neurotransmitter acetylcholine.